{
  "gene": "UniProtKB:Q5CZA5",
  "term_id": "GO:0006357",
  "term_label": "regulation of transcription by RNA polymerase II",
  "gene_symbol": "ZNF805",
  "gene_name": "Zinc finger protein 805"
}